mesodermal to mesenchymal transition involved in gastrulation [GO:0060809] (biological process) Relationships: is a type of epithelial to mesenchymal transition [GO:0001837]; is a type of embryonic morphogenesis [GO:0048598]; is part of gastrulation [GO:0007369] Sources: GOC:dph, GOC:sdb_2009, GOC:tb Definition: The epithelial to mesenchymal transition process in which a mesodermal cell loses apical/basolateral polarity, severs intercellular adhesive junctions, degrades basement membrane components and becomes a migratory mesenchymal cell as part of the process of gastrulation. Regulation: positively regulated by positive regulation of mesodermal to mesenchymal transition involved in gastrulation [GO:0060808]